{
  "term_id": "GO:0004984",
  "gene_symbol": "OR2L3",
  "gene": "UniProtKB:Q8NG85",
  "gene_name": "Olfactory receptor 2L3",
  "term_label": "olfactory receptor activity"
}